hexadecanal biosynthetic process [GO:0006634] (BP) Relationships: is a type of aldehyde biosynthetic process [GO:0046184]; is a type of hexadecanal metabolic process [GO:0046458] Also known as: hexadecanal anabolism, hexadecanal biosynthesis, hexadecanal formation, hexadecanal synthesis, palmitaldehyde biosynthesis, palmitaldehyde biosynthetic process Definition: The chemical reactions and pathways resulting in the formation of hexadecanal, the C16 straight chain aldehyde. Regulation: regulated by regulation of hexadecanal biosynthetic process [GO:1900902]; negatively regulated by negative regulation of hexadecanal biosynthetic process [GO:1900903]; positively regulated by positive regulation of hexadecanal biosynthetic process [GO:1900904] Sources: https://en.wikipedia.org/wiki/Hexadecanal